{
  "gene": "UniProtKB:Q9Y2H6",
  "term_label": "membrane",
  "gene_name": "Fibronectin type-III domain-containing protein 3A",
  "term_id": "GO:0016020",
  "gene_symbol": "FNDC3A"
}